{
  "term_label": "establishment or maintenance of cell polarity",
  "gene": "UniProtKB:Q9NPB6",
  "gene_symbol": "PARD6A",
  "gene_name": "Partitioning defective 6 homolog alpha",
  "term_id": "GO:0007163"
}